{
  "gene": "UniProtKB:P43246",
  "term_label": "somatic recombination of immunoglobulin genes involved in immune response",
  "gene_symbol": "MSH2",
  "gene_name": "DNA mismatch repair protein Msh2",
  "term_id": "GO:0002204"
}